6-deoxy-6-sulfofructose kinase activity [GO:0061594] (molecular function) Definition: Catalysis of the reaction 6-deoxy-6-sulfofructose + ATP = 6-deoxy-6-sulfofructose-1-phosphate + ADP. References: PMID:24463506 Relationships: is_a GO:0016773